{
  "gene_symbol": "ZNF579",
  "gene": "UniProtKB:Q8NAF0",
  "term_id": "UNKNOWN:0002",
  "term_label": "Unknown biological process",
  "gene_name": "Zinc finger protein 579"
}